positive regulation of neuron migration [GO:2001224] (biological process) Relationships: is_a positive regulation of cell migration [GO:0030335]; is_a regulation of neuron migration [GO:2001222]; positively regulates neuron migration [GO:0001764] Also known as: positive regulation of neuron chemotaxis, positive regulation of neuronal migration, positive regulation of neuron guidance Subtypes: positive regulation of motor neuron migration [GO:1905485] Definition: Any process that activates or increases the frequency, rate or extent of neuron migration. Sources: GOC:obol